adenylate cyclase-activating adrenergic receptor signaling pathway involved in cardiac muscle relaxation [GO:0086030] (biological process) Also known as: Gs-coupled adrenergic receptor signaling pathway involved in cardiac muscle relaxation, adrenergic receptor signaling pathway involved in cardiac muscle relaxation, adrenergic receptor signaling pathway involved in cardiac muscle relaxation via activation of AC, adrenergic receptor-induced cardiac relaxation Definition: An adrenergic receptor signaling pathway that contributes to a reduction in cardiac muscle contraction. Beta-adrenergic receptor-induced cardiac relaxation is achieved by a GPCR-activated adenylate cyclase generating cAMP; cAMP then activates the cAMP-dependent protein kinase A (PKA), which phosphorylates the sarcoplasmic reticulum (SR) membrane protein PLB. In its non-phosphorylated state, PLB acts as an inhibitor of the ATPase Ca(2+) pump of the cardiac SR (SERCA2a); inhibition of the pump is relieved upon phosphorylation. The pump removes Ca(2+) from the cytoplasm, thereby preventing cytosolic Ca(2+)-dependent activation of contractile proteins, leading to enhanced muscle relaxation. References: PMID:10571541 Sources: GOC:BHF, GOC:mtg_cardiac_conduct_nov11 Relationships: is a type of adenylate cyclase-activating adrenergic receptor signaling pathway involved in heart process [GO:0086023]; is part of relaxation of cardiac muscle [GO:0055119]